glyceraldehyde-3-phosphate metabolic process [GO:0019682] (biological process) Also known as: glyceraldehyde 3-phosphate metabolic process, glyceraldehyde 3-phosphate metabolism, glyceraldehyde-3-phosphate metabolism Subtypes: pentose-phosphate shunt, non-oxidative branch [GO:0009052], Entner-Doudoroff pathway through 6-phosphogluconate [GO:0009255], isopentenyl diphosphate biosynthetic process, methylerythritol 4-phosphate pathway [GO:0019288], GO:0019683, glyceraldehyde-3-phosphate biosynthetic process [GO:0046166], GO:0061624, Entner-Doudoroff pathway through gluconate to D-glyceraldehyde-3-phosphate [GO:0061681] Sources: GOC:ai, ISBN:0198506732 Definition: The chemical reactions and pathways involving glyceraldehyde-3-phosphate, an important intermediate in glycolysis. Relationships: is a type of aldehyde metabolic process [GO:0006081]; is_a phosphate-containing compound metabolic process [GO:0006796]; is a type of GO:0019637; is a type of carbohydrate derivative metabolic process [GO:1901135]